{
  "gene": "UniProtKB:Q8NCS4",
  "term_id": "UNKNOWN:0001",
  "gene_symbol": "TMEM35B",
  "gene_name": "Transmembrane protein 35B",
  "term_label": "Unknown molecular function"
}